negative regulation of iron ion import across plasma membrane [GO:1904439] (biological process) References: PMID:18353247 Sources: GOC:BHF, GOC:TermGenie, GOC:kom, GO_REF:0000058 Also known as: inhibition of ferrous ion import into cell, inhibition of ferrous iron import across plasma membrane, down regulation of ferrous ion import into cell, down regulation of ferrous iron import across plasma membrane, down-regulation of ferrous ion import into cell, down-regulation of ferrous iron import across plasma membrane, downregulation of ferrous ion import into cell, downregulation of ferrous iron import across plasma membrane, negative regulation of ferrous ion import into cell, negative regulation of ferrous iron import across plasma membrane, negative regulation of ferrous iron import into cell Definition: Any process that stops, prevents or reduces the frequency, rate or extent of iron ions import across plasma membrane. Relationships: is a type of negative regulation of iron ion transmembrane transport [GO:0034760]; is a type of regulation of iron ion import across plasma membrane [GO:1904438]; negatively regulates GO:0098711